nuclear membrane fusion [GO:0000740] (biological process) Definition: The joining of 2 or more lipid bilayer membranes that surround the nucleus. Sources: GOC:elh Subtypes: GO:0007086, nuclear membrane fusion involved in karyogamy [GO:0048288] Relationships: is a type of GO:0071763; is a type of organelle membrane fusion [GO:0090174]